cardioblast differentiation [GO:0010002] (biological process) Relationships: is a type of cardiocyte differentiation [GO:0035051]; is a type of stem cell differentiation [GO:0048863] Subtypes: GO:0003255, cardiac muscle cell myoblast differentiation [GO:0060379] Definition: The process in which a relatively unspecialized mesodermal cell acquires the specialized structural and/or functional features of a cardioblast. A cardioblast is a cardiac precursor cell. It is a cell that has been committed to a cardiac fate, but will undergo more cell division rather than terminally differentiating. Also known as: cardiac precursor cell differentiation, cardioblast cell differentiation, cardiomyocyte generation Regulation: regulated by regulation of cardioblast differentiation [GO:0051890]; RO_0002213 by positive regulation of cardioblast differentiation [GO:0051891]; negatively regulated by negative regulation of cardioblast differentiation [GO:0051892] Sources: GOC:go_curators